generation of neurons [GO:0048699] (BP) Definition: The process in which nerve cells are generated. This includes the production of neuroblasts and their differentiation into neurons. Also known as: neuron generation Relationships: is a type of neurogenesis [GO:0022008] Sources: GOC:nln Subtypes: forebrain generation of neurons [GO:0021872]